{
  "term_label": "cytoplasm",
  "gene": "UniProtKB:Q14444",
  "gene_name": "Caprin-1",
  "gene_symbol": "CAPRIN1",
  "term_id": "GO:0005737"
}